septal cell proliferation [GO:0022022] (biological process) Definition: The multiplication or reproduction of septal cells, resulting in the expansion of a cell population. Sources: GOC:cls, GOC:dgh, GOC:dph, GOC:jid, GO_REF:0000021 Also known as: septum cell proliferation Relationships: is a type of GO:0022012